HIR complex [GO:0000417] (cellular component) References: PMID:16303565, PMID:17180700 Sources: GOC:elh, GOC:mah Definition: A protein complex proposed to be involved in replication-independent nucleosome assembly, by promoting histone deposition onto DNA. For example, in Saccharomyces, the complex contains Hir1p, Hir2p, Hir3p, and Hpc2p. Relationships: is a type of protein-containing complex [GO:0032991] Also known as: HIRA complex